{
  "gene_symbol": "BRI3",
  "gene": "UniProtKB:O95415",
  "term_id": "UNKNOWN:0003",
  "term_label": "Unknown cellular component",
  "gene_name": "Membrane protein BRI3"
}